{
  "term_label": "nucleus",
  "gene_name": "Uncharacterized protein C19orf47",
  "term_id": "GO:0005634",
  "gene_symbol": "C19orf47",
  "gene": "UniProtKB:Q8N9M1"
}